{
  "gene": "UniProtKB:Q9Y6N7",
  "term_id": "UNKNOWN:0003",
  "gene_name": "Roundabout homolog 1",
  "term_label": "Unknown cellular component",
  "gene_symbol": "ROBO1"
}